{
  "term_label": "T cell receptor signaling pathway",
  "gene": "UniProtKB:Q6UXE8",
  "term_id": "GO:0050852",
  "gene_name": "Butyrophilin-like protein 3",
  "gene_symbol": "BTNL3"
}